paraxial mesodermal cell fate determination [GO:0048344] (biological process) Relationships: is_a GO:0007500; is part of paraxial mesodermal cell fate commitment [GO:0048343] Regulation: regulated by regulation of paraxial mesodermal cell fate determination [GO:0048345]; positively regulated by positive regulation of paraxial mesodermal cell fate determination [GO:0048346]; negatively regulated by negative regulation of paraxial mesodermal cell fate determination [GO:0048347] Definition: The process in which a cell becomes capable of differentiating autonomously into a paraxial mesoderm cell regardless of its environment; upon determination, the cell fate cannot be reversed. Sources: GOC:dgh